{
  "gene_symbol": "JADE1",
  "term_label": "histone reader activity",
  "gene": "UniProtKB:Q6IE81",
  "gene_name": "Protein Jade-1",
  "term_id": "GO:0140566"
}